cellular response to chitin [GO:0071323] (biological process) Relationships: is a type of GO:0010200; is a type of cellular response to nitrogen compound [GO:1901699]; is a type of cellular response to oxygen-containing compound [GO:1901701] Definition: Any process that results in a change in state or activity of a cell (in terms of movement, secretion, enzyme production, gene expression, etc.) as a result of a chitin stimulus. Sources: GOC:mah